cell communication involved in cardiac conduction [GO:0086065] (BP) Subtypes: cell-cell signaling involved in cardiac conduction [GO:0086019], cell communication by electrical coupling involved in cardiac conduction [GO:0086064], atrial cardiac muscle cell to AV node cell communication [GO:0086066], GO:0086067, Purkinje myocyte to ventricular cardiac muscle cell communication [GO:0086068], GO:0086069, SA node cell to atrial cardiac muscle cell communication [GO:0086070] Sources: GOC:BHF, GOC:mtg_cardiac_conduct_nov11 Relationships: is a type of cell communication [GO:0007154]; is part of cardiac conduction [GO:0061337] Definition: Any process that mediates interactions between a cell and its surroundings that contributes to the process of cardiac conduction. Encompasses interactions such as signaling or attachment between one cell and another cell, between a cell and an extracellular matrix, or between a cell and any other aspect of its environment.